{
  "gene_name": "Zinc finger protein 721",
  "gene_symbol": "ZNF721",
  "gene": "UniProtKB:Q8TF20",
  "term_label": "regulation of transcription by RNA polymerase II",
  "term_id": "GO:0006357"
}